{
  "term_id": "GO:0003713",
  "gene_symbol": "CDCA4",
  "gene_name": "Cell division cycle-associated protein 4",
  "term_label": "transcription coactivator activity",
  "gene": "UniProtKB:Q9BXL8"
}